MutLalpha complex [GO:0032389] (cellular component) Relationships: is a type of mismatch repair complex [GO:0032300]; is a type of nuclear protein-containing complex [GO:0140513] Sources: GOC:vk Definition: A heterodimer involved in the recognition of base-base and small insertion/deletion mismatches. In human the complex consists of two subunits, MLH1 and PMS2. Also known as: MMR complex, MLH1/PMS2 complex, MutL-alpha complex